{
  "gene_symbol": "RPL26L1",
  "gene_name": "Ribosomal protein uL24-like",
  "term_id": "GO:0022625",
  "gene": "UniProtKB:Q9UNX3",
  "term_label": "cytosolic large ribosomal subunit"
}